regulation of methane biosynthetic process from trimethylamine [GO:1900330] (BP) Sources: GOC:TermGenie, GOC:mengo_curators Definition: Any process that modulates the frequency, rate or extent of methane biosynthetic process from trimethylamine. Subtypes: GO:1900331, positive regulation of methane biosynthetic process from trimethylamine [GO:1900332] Relationships: is a type of regulation of amine metabolic process [GO:0033238]; is a type of GO:0043457; is a type of GO:1901577; RO_0002211 methane biosynthetic process from trimethylamine [GO:2001130]